{
  "gene": "UniProtKB:Q9NQF3",
  "term_label": "hydrolase activity",
  "gene_symbol": "SERHL",
  "term_id": "GO:0016787",
  "gene_name": "Serine hydrolase-like protein"
}